primary heart field specification [GO:0003138] (biological process) Sources: GOC:mtg_heart, GOC:rl Definition: The process that results in the delineation of a specific region of the lateral mesoderm into the area which will form the primary beating heart tube. In mammals the primary heart field gives rise to the left ventricle. Relationships: is a type of heart field specification [GO:0003128] Also known as: FHS specification, first heart field specification